{
  "gene_symbol": "CCDC107",
  "gene": "UniProtKB:Q8WV48",
  "gene_name": "Coiled-coil domain-containing protein 107",
  "term_id": "UNKNOWN:0003",
  "term_label": "Unknown cellular component"
}